{
  "gene": "UniProtKB:O95754",
  "gene_name": "Semaphorin-4F",
  "term_label": "chemorepellent activity",
  "gene_symbol": "SEMA4F",
  "term_id": "GO:0045499"
}